{
  "gene_symbol": "C4orf19",
  "term_id": "UNKNOWN:0001",
  "gene": "UniProtKB:Q8IY42",
  "gene_name": "Uncharacterized protein C4orf19",
  "term_label": "Unknown molecular function"
}